{
  "gene": "UniProtKB:Q15334",
  "gene_name": "Lethal(2) giant larvae protein homolog 1",
  "term_label": "cortical actin cytoskeleton",
  "gene_symbol": "LLGL1",
  "term_id": "GO:0030864"
}